{
  "gene": "UniProtKB:Q7Z572",
  "term_id": "UNKNOWN:0003",
  "gene_name": "Spermatogenesis-associated protein 21",
  "term_label": "Unknown cellular component",
  "gene_symbol": "SPATA21"
}